{
  "gene": "UniProtKB:Q8NHC8",
  "gene_name": "Olfactory receptor 2T6",
  "gene_symbol": "OR2T6",
  "term_id": "GO:0005886",
  "term_label": "plasma membrane"
}